{
  "term_id": "GO:0005634",
  "gene_name": "DNA-binding protein RFX7",
  "gene_symbol": "RFX7",
  "term_label": "nucleus",
  "gene": "UniProtKB:Q2KHR2"
}